{
  "gene_name": "Fumarylacetoacetase",
  "term_label": "L-tyrosine catabolic process",
  "term_id": "GO:0006572",
  "gene": "UniProtKB:P16930",
  "gene_symbol": "FAH"
}